regulation of the force of heart contraction [GO:0002026] (biological process) Relationships: is a type of GO:0008016; is a type of GO:0065008 Definition: Any process that modulates the extent of heart contraction, changing the force with which blood is propelled. Also known as: cardiac inotropy, heart inotropy Subtypes: regulation of the force of heart contraction by chemical signal [GO:0003057], regulation of the force of heart contraction by cardiac conduction [GO:0086092], positive regulation of the force of heart contraction [GO:0098735], negative regulation of the force of heart contraction [GO:0098736] References: PMID:10358008 Sources: GOC:dph, GOC:tb